{
  "gene": "UniProtKB:P43034",
  "gene_symbol": "PAFAH1B1",
  "term_label": "dynein complex binding",
  "term_id": "GO:0070840",
  "gene_name": "Platelet-activating factor acetylhydrolase IB subunit beta"
}